negative regulation of white fat cell proliferation [GO:0070351] (biological process) Sources: GOC:mah, GOC:sl Also known as: down regulation of white fat cell proliferation, down-regulation of white fat cell proliferation, downregulation of white fat cell proliferation, negative regulation of white adipocyte proliferation, negative regulation of white adipose cell proliferation, inhibition of white fat cell proliferation Relationships: is a type of GO:0070345; is a type of GO:0070350; negatively regulates GO:0070343 Definition: Any process that stops or decreases the rate or extent of white fat cell proliferation.